imaginal disc-derived male genitalia morphogenesis [GO:0048803] (biological process) Definition: The process in which the anatomical structures of male genitalia are generated and organized from the genital imaginal disc. Also known as: male genital morphogenesis Relationships: is a type of GO:0048805; is a type of male genitalia morphogenesis [GO:0048808]; is part of imaginal disc-derived male genitalia development [GO:0007485] Sources: GOC:ai, GOC:sensu